{
  "gene_symbol": "CASP10",
  "term_label": "CD95 death-inducing signaling complex",
  "term_id": "GO:0031265",
  "gene_name": "Caspase-10",
  "gene": "UniProtKB:Q92851"
}